2,2',3-trihydroxybiphenyl monooxygenase activity [GO:0102325] (molecular function) Definition: Catalysis of the reaction: biphenyl-2,2',3-triol + O2 + NADH + H+ = 2,2',3,3'-tetrahydroxybiphenyl + NAD + H2O. Sources: GOC:pz, RHEA:63516 Relationships: is a type of GO:0016709